{
  "term_id": "GO:0019104",
  "term_label": "DNA N-glycosylase activity",
  "gene_symbol": "NEIL3",
  "gene_name": "Endonuclease 8-like 3",
  "gene": "UniProtKB:Q8TAT5"
}